regulation of double-strand break repair via nonhomologous end joining [GO:2001032] (biological process) Definition: Any process that modulates the frequency, rate or extent of double-strand break repair via nonhomologous end joining. Relationships: is a type of regulation of double-strand break repair [GO:2000779]; RO_0002211 double-strand break repair via nonhomologous end joining [GO:0006303] Also known as: regulation of NHEJ Sources: GOC:obol Subtypes: negative regulation of double-strand break repair via nonhomologous end joining [GO:2001033], GO:2001034